{
  "term_id": "GO:0045503",
  "term_label": "dynein light chain binding",
  "gene_symbol": "DNAI3",
  "gene": "UniProtKB:Q8IWG1",
  "gene_name": "Dynein axonemal intermediate chain 3"
}